{
  "term_label": "vesicle-mediated transport",
  "term_id": "GO:0016192",
  "gene_name": "ADP-ribosylation factor-like protein 1",
  "gene_symbol": "ARL1",
  "gene": "UniProtKB:P40616"
}